{
  "gene": "UniProtKB:P0C870",
  "term_id": "GO:0005737",
  "gene_name": "Bifunctional peptidase and (3S)-lysyl hydroxylase JMJD7",
  "gene_symbol": "JMJD7",
  "term_label": "cytoplasm"
}